{
  "term_label": "vacuolar membrane",
  "gene": "UniProtKB:Q6PJI9",
  "gene_name": "GATOR complex protein WDR59",
  "gene_symbol": "WDR59",
  "term_id": "GO:0005774"
}